{
  "gene_symbol": "EHBP1",
  "term_id": "GO:0030036",
  "term_label": "actin cytoskeleton organization",
  "gene_name": "EH domain-binding protein 1",
  "gene": "UniProtKB:Q8NDI1"
}